{
  "term_id": "GO:0003723",
  "gene_symbol": "RPL7A",
  "gene": "UniProtKB:P62424",
  "gene_name": "Large ribosomal subunit protein eL8",
  "term_label": "RNA binding"
}